meristem determinacy [GO:0010022] (biological process) Relationships: is a type of multicellular organismal process [GO:0032501]; BFO_0000050 GO:0010073 Definition: The process in which a meristem becomes determinate (i.e. ceases to produce lateral organs and may or may not terminally differentiate). Subtypes: floral meristem determinacy [GO:0010582] Sources: GOC:lr